{
  "term_id": "GO:0071051",
  "term_label": "poly(A)-dependent snoRNA 3'-end processing",
  "gene": "UniProtKB:Q01780",
  "gene_name": "Exosome component 10",
  "gene_symbol": "EXOSC10"
}